{
  "term_id": "GO:0000774",
  "gene_symbol": "HSPA4L",
  "gene_name": "Heat shock 70 kDa protein 4L",
  "gene": "UniProtKB:O95757",
  "term_label": "adenyl-nucleotide exchange factor activity"
}